{
  "term_id": "GO:0016082",
  "gene": "UniProtKB:Q5SQN1",
  "term_label": "synaptic vesicle priming",
  "gene_name": "Synaptosomal-associated protein 47",
  "gene_symbol": "SNAP47"
}